{
  "gene": "UniProtKB:Q13144",
  "term_id": "UNKNOWN:0002",
  "gene_symbol": "EIF2B5",
  "term_label": "Unknown biological process",
  "gene_name": "Translation initiation factor eIF-2B subunit epsilon"
}